{
  "gene": "UniProtKB:Q3T906",
  "term_id": "GO:0003976",
  "gene_name": "N-acetylglucosamine-1-phosphotransferase subunits alpha_beta",
  "gene_symbol": "GNPTAB",
  "term_label": "UDP-N-acetylglucosamine-lysosomal-enzyme N-acetylglucosaminephosphotransferase activity"
}